{
  "gene": "UniProtKB:Q5R3F8",
  "term_label": "signaling receptor activity",
  "term_id": "GO:0038023",
  "gene_name": "Protein phosphatase 1 regulatory subunit 29",
  "gene_symbol": "ELFN2"
}